{
  "gene": "UniProtKB:Q8NCN4",
  "gene_symbol": "RNF169",
  "term_label": "ubiquitin-protein transferase activity",
  "term_id": "GO:0004842",
  "gene_name": "E3 ubiquitin-protein ligase RNF169"
}